{
  "term_label": "myosin filament",
  "gene": "UniProtKB:P13535",
  "gene_name": "Myosin-8",
  "gene_symbol": "MYH8",
  "term_id": "GO:0032982"
}